{
  "term_id": "UNKNOWN:0001",
  "gene": "UniProtKB:O14994",
  "term_label": "Unknown molecular function",
  "gene_name": "Synapsin-3",
  "gene_symbol": "SYN3"
}